detection of muscle inactivity [GO:0014869] (biological process) Sources: GOC:mtg_muscle Relationships: is a type of detection of inactivity [GO:0014863]; is a type of response to muscle inactivity [GO:0014870] Subtypes: detection of muscle inactivity involved in regulation of muscle adaptation [GO:0014884] Definition: The series of events in which a muscle inactivity stimulus is received by a cell and converted into a molecular signal.